{
  "term_label": "cell adhesion molecule binding",
  "gene": "UniProtKB:Q9UN73",
  "gene_name": "Protocadherin alpha-6",
  "term_id": "GO:0050839",
  "gene_symbol": "PCDHA6"
}